{
  "gene_name": "Secreted frizzled-related protein 3",
  "gene": "UniProtKB:Q92765",
  "gene_symbol": "FRZB",
  "term_id": "GO:0035567",
  "term_label": "non-canonical Wnt signaling pathway"
}